bile acid:sodium symporter activity [GO:0008508] (molecular function) Also known as: sodium/bile acid symporter activity Relationships: is a type of bile acid transmembrane transporter activity [GO:0015125]; is a type of GO:0140161 Definition: Enables the transfer of a solute or solutes from one side of a membrane to the other according to the reaction: bile acid(out) + Na+(out) = bile acid(in) + Na+(in). Sources: TC:2.A.28.-.-